MAPK cascade [GO:0000165] (biological process) Definition: An intracellular protein kinase cascade containing at least a MAP kinase (MAPK). It starts with the activation of a MAP3K, and the consecutive activation of a MPK2K and a MAPK. The cascade can also contain an additional tier: the upstream MAP4K. The kinases in each tier phosphorylate and activate the kinase in the downstream tier to transmit a signal within a cell. Note: MAPK cascades lie downstream of many cell surface receptors and cooperate in transmitting various extracellular signals to the nucleus. One way by which the specificity of each cascade is regulated is through the existence of several distinct components in each tier of the different cascades. The cascades are typically named according to the component in the MAPK tier. Also known as: MAP kinase cascade, MAP kinase kinase kinase cascade, MAPK signal transduction, MAPKKK cascade, mitogen-activated protein kinase cascade, ERK/MAPK cascade, MAPKKK cascade during sporulation, MAPK signaling, MAPK signalling Relationships: is_a intracellular signaling cassette [GO:0141124] Subtypes: JNK cascade [GO:0007254], p38MAPK cascade [GO:0038066], stress-activated MAPK cascade [GO:0051403], GO:0070371, ERK5 cascade [GO:0070375], GO:0071507 Regulation: regulated by regulation of MAPK cascade [GO:0043408]; negatively regulated by negative regulation of MAPK cascade [GO:0043409]; positively regulated by positive regulation of MAPK cascade [GO:0043410] References: PMID:20811974, PMID:9561267